{
  "term_label": "neurotransmitter receptor activity",
  "term_id": "GO:0030594",
  "gene_symbol": "HTR2C",
  "gene_name": "5-hydroxytryptamine receptor 2C",
  "gene": "UniProtKB:P28335"
}